oxidoreductase activity, acting on phosphorus or arsenic in donors, disulfide as acceptor [GO:0030614] (molecular function) Also known as: oxidoreductase activity, acting on phosphorus or arsenic in donors, with disulphide as acceptor Definition: Catalysis of an oxidation-reduction (redox) reaction in which a phosphorus- or arsenic-containing group acts as a hydrogen or electron donor and reduces a disulfide. Relationships: is a type of GO:0030613 Sources: GOC:mah Subtypes: arsenate reductase (glutaredoxin) activity [GO:0008794], arsenate reductase (thioredoxin) activity [GO:0030612], methylarsonate reductase activity [GO:0050610]